{
  "gene_name": "Putative protein SEM1, isoform 2",
  "term_label": "double-strand break repair via homologous recombination",
  "term_id": "GO:0000724",
  "gene_symbol": "SEM1",
  "gene": "UniProtKB:Q6ZVN7"
}